{
  "term_label": "regulation of cell migration",
  "gene": "UniProtKB:P61278",
  "gene_name": "Somatostatin",
  "gene_symbol": "SST",
  "term_id": "GO:0030334"
}